phosphopantetheine binding [GO:0031177] (molecular function) Definition: Binding to phosphopantetheine, the vitamin pantetheine 4'-(dihydrogen phosphate). Sources: GOC:mah, GOC:vw Relationships: is a type of GO:0019842; is a type of GO:0033218; is a type of modified amino acid binding [GO:0072341]